{
  "term_id": "GO:0030889",
  "gene_symbol": "TNFRSF21",
  "gene": "UniProtKB:O75509",
  "gene_name": "Tumor necrosis factor receptor superfamily member 21",
  "term_label": "negative regulation of B cell proliferation"
}